{
  "term_label": "manganese ion transport",
  "gene_name": "Calcium_manganese antiporter SLC30A10",
  "gene_symbol": "SLC30A10",
  "gene": "UniProtKB:Q6XR72",
  "term_id": "GO:0006828"
}